{
  "gene": "UniProtKB:Q14241",
  "gene_name": "Elongin-A",
  "gene_symbol": "ELOA",
  "term_label": "Unknown cellular component",
  "term_id": "UNKNOWN:0003"
}